alpha-santonin 1,2-reductase activity [GO:0047659] (molecular function) Definition: Catalysis of the reaction: 1,2-dihydrosantonin + NAD(P)+ = alpha-santonin + NAD(P)H + H+. Also known as: a-santonin 1,2-reductase activity, 1,2-dihydrosantonin:NAD(P)+ 1,2-oxidoreductase activity Sources: EC:1.3.1.47, MetaCyc:ALPHA-SANTONIN-12-REDUCTASE-RXN Relationships: is a type of oxidoreductase activity, acting on the CH-CH group of donors, NAD or NADP as acceptor [GO:0016628]